{
  "gene_symbol": "RANBP3L",
  "gene_name": "Ran-binding protein 3-like",
  "gene": "UniProtKB:Q86VV4",
  "term_label": "protein export from nucleus",
  "term_id": "GO:0006611"
}